{
  "term_label": "Unknown cellular component",
  "gene_symbol": "LINC01590",
  "gene": "UniProtKB:Q5TEZ4",
  "term_id": "UNKNOWN:0003",
  "gene_name": "Putative uncharacterized protein encoded by LINC01590"
}